Bcl3-Bcl10 complex [GO:0032996] (cellular component) References: PMID:16280327 Relationships: is a type of intracellular protein-containing complex [GO:0140535] Definition: A protein complex containing Bcl3 and Bcl10, which forms when Akt1 is activated by TNF-alpha to phosphorylate Bcl10; the Bcl3-Bcl10 complex is translocated to the nucleus.